{
  "gene": "UniProtKB:Q9BT67",
  "term_label": "ubiquitin-dependent protein catabolic process",
  "gene_symbol": "NDFIP1",
  "term_id": "GO:0006511",
  "gene_name": "NEDD4 family-interacting protein 1"
}